{
  "term_label": "Unknown molecular function",
  "gene_symbol": "FMN2",
  "gene_name": "Formin-2",
  "gene": "UniProtKB:Q9NZ56",
  "term_id": "UNKNOWN:0001"
}